adult walking behavior [GO:0007628] (biological process) Definition: The behavior of an adult relating to the progression of that organism along the ground by the process of lifting and setting down each leg. Relationships: is_a adult locomotory behavior [GO:0008344]; is a type of walking behavior [GO:0090659] Sources: GOC:jid, GOC:pr, ISBN:0198606907 Also known as: adult walking behaviour